{
  "gene_name": "Nuclear factor of activated T-cells, cytoplasmic 4",
  "gene_symbol": "NFATC4",
  "term_id": "GO:0005634",
  "term_label": "nucleus",
  "gene": "UniProtKB:Q14934"
}